{
  "term_label": "transforming growth factor beta receptor signaling pathway",
  "term_id": "GO:0007179",
  "gene_name": "Transforming growth factor beta-2 proprotein",
  "gene": "UniProtKB:P61812",
  "gene_symbol": "TGFB2"
}